midbrain morphogenesis [GO:1904693] (biological process) Definition: The developmental process by which a midbrain is generated and organized. Relationships: is a type of GO:0009653; is part of midbrain development [GO:0030901]; BFO_0000050 brain morphogenesis [GO:0048854] References: PMID:21347250 Sources: GOC:PARL, GOC:TermGenie, GOC:bf, GO_REF:0000083 Also known as: MB morphogenesis, mesencephalon morphogenesis